{
  "term_id": "UNKNOWN:0002",
  "gene_name": "Pecanex-like protein 3",
  "term_label": "Unknown biological process",
  "gene": "UniProtKB:Q9H6A9",
  "gene_symbol": "PCNX3"
}